{
  "term_label": "negative regulation of signal transduction",
  "term_id": "GO:0009968",
  "gene_symbol": "INPP5D",
  "gene": "UniProtKB:Q92835",
  "gene_name": "Phosphatidylinositol 3,4,5-trisphosphate 5-phosphatase 1"
}